{
  "gene_symbol": "KRTAP4-7",
  "gene_name": "Keratin-associated protein 4-7",
  "term_id": "UNKNOWN:0003",
  "term_label": "Unknown cellular component",
  "gene": "UniProtKB:Q9BYR0"
}